{
  "gene_symbol": "GJA5",
  "gene": "UniProtKB:P36382",
  "gene_name": "Gap junction alpha-5 protein",
  "term_id": "GO:0086076",
  "term_label": "gap junction channel activity involved in atrial cardiac muscle cell-AV node cell electrical coupling"
}